{
  "gene": "UniProtKB:P14151",
  "term_label": "sialic acid binding",
  "gene_symbol": "SELL",
  "term_id": "GO:0033691",
  "gene_name": "L-selectin"
}